netrin-activated signaling pathway [GO:0038007] (biological process) Relationships: is a type of GO:0007166 Also known as: netrin signaling pathway, netrin-activated signal transduction pathway, netrin-activated signalling pathway, netrin-mediated signaling pathway Definition: The series of molecular signals initiated by the binding of a netrin protein to its receptor on the surface of the target cell, and ending with the regulation of a downstream cellular process, e.g. transcription. Netrins can act as chemoattractant signals for some cells and chemorepellent signals for others. Netrins also have roles outside of cell and axon guidance. References: PMID:10399919, PMID:15960985, PMID:19785719, PMID:20108323 Sources: GOC:signaling Regulation: regulated by regulation of netrin-activated signaling pathway [GO:1902841]; negatively regulated by negative regulation of netrin-activated signaling pathway [GO:1902842]; positively regulated by positive regulation of netrin-activated signaling pathway [GO:1902843]